positive regulation of CD8-positive, alpha-beta T cell extravasation [GO:2000451] (biological process) Definition: Any process that activates or increases the frequency, rate or extent of CD8-positive, alpha-beta T cell extravasation. Sources: GOC:obol Relationships: is a type of positive regulation of T cell extravasation [GO:2000409]; is a type of regulation of CD8-positive, alpha-beta T cell extravasation [GO:2000449]; positively regulates CD8-positive, alpha-beta T cell extravasation [GO:0035697] Subtypes: GO:2000454, positive regulation of T-helper 17 cell extravasation [GO:2000457]